tetraterpenoid biosynthetic process [GO:0016109] (biological process) Definition: The chemical reactions and pathways resulting in the formation of tetraterpenoid compounds, terpenoids with eight isoprene units. Sources: GOC:go_curators Also known as: tetraterpenoid anabolism, tetraterpenoid biosynthesis, tetraterpenoid formation, tetraterpenoid synthesis, tetraterpene biosynthesis, tetraterpene biosynthetic process Relationships: is a type of GO:0016114 Subtypes: carotenoid biosynthetic process [GO:0016117]